{
  "term_label": "Unknown biological process",
  "gene_name": "Elongin-B",
  "term_id": "UNKNOWN:0002",
  "gene_symbol": "ELOB",
  "gene": "UniProtKB:Q15370"
}